regulation of metanephric glomerulus development [GO:0072298] (biological process) Sources: GOC:mtg_kidney_jan10 Subtypes: negative regulation of metanephric glomerulus development [GO:0072299], positive regulation of metanephric glomerulus development [GO:0072300] Definition: Any process that modulates the rate, frequency or extent of metanephric glomerulus development, the progression of the metanephric glomerulus over time from its initial formation until its mature state. The metanephric glomerulus is a capillary tuft surrounded by Bowman's capsule in nephrons of the vertebrate kidney, or metanephros. Relationships: is a type of metanephros development [GO:0001656]; is a type of regulation of glomerulus development [GO:0090192]; regulates metanephric glomerulus development [GO:0072224]